{
  "gene_symbol": "JOSD1",
  "term_id": "UNKNOWN:0002",
  "term_label": "Unknown biological process",
  "gene": "UniProtKB:Q15040",
  "gene_name": "Josephin-1"
}